{
  "term_id": "UNKNOWN:0001",
  "gene_symbol": "EXOC1L",
  "term_label": "Unknown molecular function",
  "gene_name": "Exocyst complex component 1-like",
  "gene": "UniProtKB:A0A1B0GW35"
}